{
  "term_id": "GO:0016167",
  "gene_symbol": "GFRA4",
  "gene_name": "GDNF family receptor alpha-4",
  "term_label": "glial cell-derived neurotrophic factor receptor activity",
  "gene": "UniProtKB:Q9GZZ7"
}